{
  "gene": "UniProtKB:A6NC57",
  "term_label": "Unknown cellular component",
  "gene_name": "Ankyrin repeat domain-containing protein 62",
  "gene_symbol": "ANKRD62",
  "term_id": "UNKNOWN:0003"
}